{
  "gene": "UniProtKB:Q8NGQ3",
  "gene_name": "Olfactory receptor 1S2",
  "gene_symbol": "OR1S2",
  "term_label": "signal transduction",
  "term_id": "GO:0007165"
}